{
  "term_id": "GO:0007218",
  "term_label": "neuropeptide signaling pathway",
  "gene_name": "G-protein coupled receptor 83",
  "gene_symbol": "GPR83",
  "gene": "UniProtKB:Q9NYM4"
}